{
  "gene": "UniProtKB:Q9P266",
  "gene_symbol": "JCAD",
  "gene_name": "Junctional cadherin 5-associated protein",
  "term_id": "GO:1903589",
  "term_label": "positive regulation of blood vessel endothelial cell proliferation involved in sprouting angiogenesis"
}